homoserine O-acetyltransferase activity [GO:0004414] (molecular function) Relationships: is a type of O-acetyltransferase activity [GO:0016413] Also known as: homoserine transacetylase activity, L-homoserine O-acetyltransferase activity, acetyl-CoA:L-homoserine O-acetyltransferase activity, homoserine O-trans-acetylase activity, homoserine acetyltransferase activity, homoserine-O-transacetylase activity Definition: Catalysis of the reaction: L-homoserine + acetyl-CoA = O-acetyl-L-homoserine + CoA. Sources: EC:2.3.1.31, RHEA:13701